{
  "gene_symbol": "FAM180B",
  "gene": "UniProtKB:Q6P0A1",
  "term_label": "Unknown molecular function",
  "term_id": "UNKNOWN:0001",
  "gene_name": "Protein FAM180B"
}